{
  "term_id": "GO:0000981",
  "gene": "UniProtKB:P11161",
  "gene_symbol": "EGR2",
  "gene_name": "E3 SUMO-protein ligase EGR2",
  "term_label": "DNA-binding transcription factor activity, RNA polymerase II-specific"
}